{
  "gene": "UniProtKB:Q9Y2W3",
  "gene_symbol": "SLC45A1",
  "term_label": "sucrose:proton symporter activity",
  "term_id": "GO:0008506",
  "gene_name": "Proton-associated sugar transporter A"
}